{
  "term_id": "UNKNOWN:0003",
  "gene": "UniProtKB:Q5VT40",
  "gene_name": "Protein FAM78B",
  "gene_symbol": "FAM78B",
  "term_label": "Unknown cellular component"
}